meiotic DNA double-strand break formation [GO:0042138] (biological process) Definition: The cell cycle process in which double-strand breaks are generated at defined hotspots throughout the genome during meiosis I. This results in the initiation of meiotic recombination. Subtypes: meiotic DNA double-strand break formation involved in reciprocal meiotic recombination [GO:0010780], meiotic DNA double-strand break formation involved in meiotic gene conversion [GO:0010781] Regulation: regulated by regulation of meiotic DNA double-strand break formation [GO:1903341]; negatively regulated by negative regulation of meiotic DNA double-strand break formation [GO:1903342]; positively regulated by positive regulation of meiotic DNA double-strand break formation [GO:1903343] References: PMID:11529427 Sources: GOC:elh, GOC:jl Relationships: is a type of DNA metabolic process [GO:0006259]; is a type of meiosis I cell cycle process [GO:0061982]